{
  "term_label": "neural crest cell migration",
  "gene_name": "Semaphorin-4G",
  "gene_symbol": "SEMA4G",
  "term_id": "GO:0001755",
  "gene": "UniProtKB:Q9NTN9"
}